{
  "gene": "UniProtKB:Q9UFW8",
  "term_label": "nucleus",
  "gene_name": "CGG triplet repeat-binding protein 1",
  "term_id": "GO:0005634",
  "gene_symbol": "CGGBP1"
}